fibroblast growth factor receptor antagonist activity [GO:0030353] (molecular function) Also known as: FGF receptor antagonist activity, FGFR antagonist activity Relationships: is_a fibroblast growth factor receptor binding [GO:0005104]; is_a receptor antagonist activity [GO:0048019]; is part of GO:0040037 Sources: GOC:mah Definition: Interacts with the fibroblast growth factor receptor to reduce the action of another ligand, the agonist.